{
  "term_id": "GO:0010507",
  "gene": "UniProtKB:Q7L523",
  "gene_name": "Ras-related GTP-binding protein A",
  "term_label": "negative regulation of autophagy",
  "gene_symbol": "RRAGA"
}